dihydrofolate reductase activity [GO:0004146] (molecular function) Also known as: dihydrofolate reduction, 5,6,7,8-tetrahydrofolate:NADP+ oxidoreductase activity, 7,8-dihydrofolate reductase activity, DHFR, NADPH-dihydrofolate reductase activity, dihydrofolate reductase:thymidylate synthase activity, dihydrofolic acid reductase activity, dihydrofolic reductase activity, folic acid reductase activity, folic reductase activity, pteridine reductase:dihydrofolate reductase activity, tetrahydrofolate dehydrogenase activity, thymidylate synthetase-dihydrofolate reductase activity Relationships: is a type of oxidoreductase activity, acting on the CH-NH group of donors, NAD or NADP as acceptor [GO:0016646] Definition: Catalysis of the reaction: 5,6,7,8-tetrahydrofolate + NADP+ = 7,8-dihydrofolate + NADPH + H+. Sources: EC:1.5.1.3